cranial ganglion morphogenesis [GO:0061559] (biological process) Definition: The process in which the anatomical structure of a cranial ganglion is generated and organized. Subtypes: trigeminal ganglion morphogenesis [GO:0061556], facioacoustic ganglion morphogenesis [GO:1904836] Sources: GOC:dph Also known as: cranial ganglia morphogenesis Relationships: is a type of ganglion morphogenesis [GO:0061552]; is part of cranial nerve morphogenesis [GO:0021602]; is part of GO:0061550